{
  "gene": "UniProtKB:Q96MK2",
  "term_label": "Unknown molecular function",
  "term_id": "UNKNOWN:0001",
  "gene_name": "RIPOR family member 3",
  "gene_symbol": "RIPOR3"
}